{
  "gene_name": "Immunoglobulin heavy variable 3-66",
  "gene": "UniProtKB:A0A0C4DH42",
  "term_label": "immunoglobulin mediated immune response",
  "gene_symbol": "IGHV3-66",
  "term_id": "GO:0016064"
}